retina morphogenesis in camera-type eye [GO:0060042] (biological process) Relationships: is a type of anatomical structure morphogenesis [GO:0009653]; is part of camera-type eye morphogenesis [GO:0048593]; is part of GO:0060041 Definition: The process in which the anatomical structure of the retina is generated and organized. Sources: GOC:bf, GOC:dph, GOC:mtg_sensu Also known as: retina morphogenesis in camera-style eye, retinogenesis